somatic ring canal [GO:0098549] (cellular component) Definition: A stable intercellular bridge between somatic cells. Examples include the intercellular bridges between ovarian follicle cells in insects and between imaginal disc cells in insects. References: PMID:22135360, PMID:670316 Sources: GOC:dos Relationships: is a type of GO:0045171